{
  "gene_symbol": "DIPK1B",
  "gene": "UniProtKB:Q5VUD6",
  "term_label": "Unknown molecular function",
  "term_id": "UNKNOWN:0001",
  "gene_name": "Divergent protein kinase domain 1B"
}